{
  "gene_name": "D site-binding protein",
  "term_id": "GO:0000978",
  "term_label": "RNA polymerase II cis-regulatory region sequence-specific DNA binding",
  "gene": "UniProtKB:Q10586",
  "gene_symbol": "DBP"
}